tartrate catabolic process [GO:1901276] (biological process) Definition: The chemical reactions and pathways resulting in the breakdown of tartrate. Relationships: is a type of catabolic process [GO:0009056]; is a type of GO:1901275 Also known as: tartrate breakdown, tartrate catabolism, tartrate degradation Sources: GOC:TermGenie, GOC:yaf, UniPathway:UPA00839